{
  "term_id": "GO:0004930",
  "gene_symbol": "S1PR5",
  "gene_name": "Sphingosine 1-phosphate receptor 5",
  "gene": "UniProtKB:Q9H228",
  "term_label": "G protein-coupled receptor activity"
}